{
  "term_label": "cilium assembly",
  "gene_symbol": "TEKT2",
  "gene": "UniProtKB:Q9UIF3",
  "term_id": "GO:0060271",
  "gene_name": "Tektin-2"
}